radial glia guided migration of cerebellar granule cell [GO:0021933] (biological process) References: PMID:15157725 Sources: GOC:cls, GOC:dgh, GOC:dph, GOC:jid, GO_REF:0000021 Relationships: is a type of GO:0021932 Definition: The inward migration of postmitotic granule cells along a radial glial cell from the external granule layer to the internal granule cell layer.